phosphatidylinositol lysophospholipase activity [GO:0120561] (molecular function) Sources: RHEA:32987 Definition: Catalysis of the reaction: a 1-acyl-sn-glycero-3-phospho-(1D-myo-inositol) + H2O = sn-glycero-3-phospho-1D-myo-inositol + a fatty acid + H+. Relationships: is a type of lysophospholipase activity [GO:0120558]